{
  "gene_name": "Primary cilium assembly protein FAM149B1",
  "gene": "UniProtKB:Q96BN6",
  "gene_symbol": "FAM149B1",
  "term_label": "cilium assembly",
  "term_id": "GO:0060271"
}